{
  "term_id": "GO:0051010",
  "gene": "UniProtKB:Q96DZ5",
  "term_label": "microtubule plus-end binding",
  "gene_name": "CAP-Gly domain-containing linker protein 3",
  "gene_symbol": "CLIP3"
}